{
  "gene": "UniProtKB:Q6ZVL8",
  "gene_symbol": "Q6ZVL8",
  "term_label": "Unknown biological process",
  "gene_name": "Putative uncharacterized protein FLJ42384",
  "term_id": "UNKNOWN:0002"
}